{
  "gene_name": "Large neutral amino acids transporter small subunit 4",
  "gene_symbol": "SLC43A2",
  "term_label": "Unknown cellular component",
  "term_id": "UNKNOWN:0003",
  "gene": "UniProtKB:Q8N370"
}